pyridoxal phosphate biosynthetic process from pyridoxamine [GO:0010144] (biological process) Relationships: is a type of GO:0009443; is a type of pyridoxamine metabolic process [GO:0042818] Sources: GOC:pz Definition: The chemical reactions and pathways resulting in the formation of pyridoxal phosphate, the active form of vitamin B6, from pyridoxamine. Also known as: pyridoxal 5'-phosphate salvage from pyridoxamine, pyridoxal phosphate anabolism from pyridoxamine, pyridoxal phosphate formation from pyridoxamine, pyridoxal phosphate synthesis from pyridoxamine, vitamin B6 biosynthesis from pyridoxamine, vitamin B6 biosynthetic process from pyridoxamine